{
  "gene": "UniProtKB:A0A087WXM9",
  "gene_name": "Meiosis-specific kinetochore protein",
  "term_id": "GO:0016321",
  "gene_symbol": "MEIKIN",
  "term_label": "female meiosis chromosome segregation"
}